{
  "gene_name": "Probable ubiquitin carboxyl-terminal hydrolase FAF-X",
  "term_id": "GO:0005634",
  "term_label": "nucleus",
  "gene": "UniProtKB:Q93008",
  "gene_symbol": "USP9X"
}